{
  "gene_name": "G protein-activated inward rectifier potassium channel 4",
  "term_label": "plasma membrane",
  "term_id": "GO:0005886",
  "gene": "UniProtKB:P48544",
  "gene_symbol": "KCNJ5"
}